regulation of interleukin-17 production [GO:0032660] (biological process) Definition: Any process that modulates the frequency, rate, or extent of production of any member of the interleukin-17 family of cytokines. References: PMID:16482511 Sources: GOC:add, GOC:mah Also known as: regulation of CTLA-8 production, regulation of Cytotoxic T-lymphocyte-associated antigen 8 secretion, regulation of IL-17 production, regulation of interleukin-17 biosynthetic process, regulation of interleukin-17 secretion Relationships: is a type of regulation of cytokine production [GO:0001817]; regulates GO:0032620 Subtypes: negative regulation of interleukin-17 production [GO:0032700], positive regulation of interleukin-17 production [GO:0032740], regulation of interleukin-17A production [GO:0150151]